{
  "term_id": "GO:0000981",
  "term_label": "DNA-binding transcription factor activity, RNA polymerase II-specific",
  "gene_symbol": "ZNF322",
  "gene_name": "Zinc finger protein 322",
  "gene": "UniProtKB:Q6U7Q0"
}